regulation of nuclear receptor-mediated glucocorticoid signaling pathway [GO:2000322] (biological process) Sources: GOC:BHF Relationships: is a type of regulation of intracellular steroid hormone receptor signaling pathway [GO:0033143]; RO_0002211 nuclear receptor-mediated glucocorticoid signaling pathway [GO:0042921] Also known as: regulation of glucocorticoid receptor signaling pathway, regulation of glucocorticoid receptor signalling pathway Subtypes: negative regulation of nuclear receptor-mediated glucocorticoid signaling pathway [GO:2000323], positive regulation of nuclear receptor-mediated glucocorticoid signaling pathway [GO:2000324] Definition: Any process that modulates the frequency, rate or extent of nuclear receptor-mediated glucocorticoid signaling pathway.